{
  "gene": "UniProtKB:Q70HW3",
  "term_label": "S-adenosyl-L-methionine transmembrane transporter activity",
  "term_id": "GO:0000095",
  "gene_symbol": "SLC25A26",
  "gene_name": "Mitochondrial S-adenosylmethionine carrier protein"
}